L-ascorbic acid biosynthetic process via GDP-alpha-D-mannose [GO:0090531] (biological process) Also known as: L-ascorbic acid biosynthesis via GDP-alpha-D-mannose, Smirnoff-Wheeler's pathway Definition: The chemical reactions and pathways resulting in the formation of L-ascorbic acid via the intermediate GDP-alpha-D-mannose. References: PMID:11153268 Sources: MetaCyc:PWY-882 Relationships: is a type of L-ascorbic acid biosynthetic process [GO:0019853]